{
  "gene": "UniProtKB:P80217",
  "gene_name": "Interferon-induced 35 kDa protein",
  "gene_symbol": "IFI35",
  "term_label": "nucleus",
  "term_id": "GO:0005634"
}